{
  "gene_name": "Uncharacterized protein C2orf74",
  "term_id": "UNKNOWN:0003",
  "gene": "UniProtKB:A8MZ97",
  "gene_symbol": "C2orf74",
  "term_label": "Unknown cellular component"
}